2-polyprenyl-6-hydroxyphenol O-methyltransferase activity [GO:1990888] (MF) Relationships: is a type of O-methyltransferase activity [GO:0008171] Definition: Catalysis of the reaction: 2-polyprenyl-6-hydroxyphenol + S-adenosyl-L-methionine = 2-polyprenyl-6-methoxyphenol + S-adenosyl-L-homocysteine + H+. References: PMID:10419476